excitatory neuromuscular junction of somatic myotube [GO:0098525] (cellular component) Definition: A neuromuscular junction that functions in the excitation of somatic muscle myotubes, such as an arthropod somatic muscle cells. Sources: GOC:dos Relationships: is a type of excitatory neuromuscular junction [GO:0098520]; is a type of neuromuscular junction of somatic muscle myotube [GO:0098524]